{
  "gene": "UniProtKB:Q9P291",
  "gene_name": "Armadillo repeat-containing X-linked protein 1",
  "term_label": "Unknown molecular function",
  "gene_symbol": "ARMCX1",
  "term_id": "UNKNOWN:0001"
}